{
  "gene": "UniProtKB:Q8NCF0",
  "gene_name": "C-type lectin domain family 18 member C",
  "term_id": "UNKNOWN:0002",
  "gene_symbol": "CLEC18C",
  "term_label": "Unknown biological process"
}